ubiquitin-ubiquitin ligase activity [GO:0034450] (molecular function) Definition: Isoenergetic transfer of ubiquitin from one protein to an existing ubiquitin chain via the reaction X-ubiquitin + Y-ubiquitin = Y-ubiquitin-ubiquitin + X, where both the X-ubiquitin and Y-ubiquitin-ubiquitin linkages are thioester bonds between the C-terminal glycine of ubiquitin and a sulfhydryl side group of a cysteine residue. Also known as: E4 References: PMID:10089879, PMID:17190603 Sources: GOC:mah, GOC:mcc Relationships: is a type of GO:0061630